{
  "term_id": "GO:0000122",
  "gene_symbol": "ZBTB2",
  "gene_name": "Zinc finger and BTB domain-containing protein 2",
  "term_label": "negative regulation of transcription by RNA polymerase II",
  "gene": "UniProtKB:Q8N680"
}